{
  "gene": "UniProtKB:Q5JTD0",
  "gene_name": "Tight junction-associated protein 1",
  "gene_symbol": "TJAP1",
  "term_label": "Unknown molecular function",
  "term_id": "UNKNOWN:0001"
}